{
  "gene": "UniProtKB:Q99706",
  "term_id": "GO:0032394",
  "gene_symbol": "KIR2DL4",
  "gene_name": "Killer cell immunoglobulin-like receptor 2DL4",
  "term_label": "MHC class Ib receptor activity"
}